{
  "gene_symbol": "SLC17A9",
  "term_label": "ATP transport",
  "gene_name": "Voltage-gated purine nucleotide uniporter SLC17A9",
  "term_id": "GO:0015867",
  "gene": "UniProtKB:Q9BYT1"
}